{
  "gene": "UniProtKB:Q9UKC9",
  "gene_name": "F-box_LRR-repeat protein 2",
  "gene_symbol": "FBXL2",
  "term_id": "GO:1990756",
  "term_label": "ubiquitin-like ligase-substrate adaptor activity"
}